{
  "term_id": "UNKNOWN:0001",
  "gene": "UniProtKB:Q9H6K5",
  "gene_name": "Proline-rich protein 36",
  "term_label": "Unknown molecular function",
  "gene_symbol": "PRR36"
}